{
  "term_id": "UNKNOWN:0001",
  "term_label": "Unknown molecular function",
  "gene": "UniProtKB:Q6ZMU1",
  "gene_symbol": "C3P1",
  "gene_name": "Putative protein C3P1"
}